{
  "term_id": "GO:0004521",
  "gene_symbol": "ENDOG",
  "gene_name": "Endonuclease G, mitochondrial",
  "gene": "UniProtKB:Q14249",
  "term_label": "RNA endonuclease activity"
}